{
  "gene": "UniProtKB:A8K010",
  "term_label": "Unknown cellular component",
  "gene_name": "Putative transcriptional regulator encoded by LINC00473",
  "gene_symbol": "LINC00473",
  "term_id": "UNKNOWN:0003"
}